{
  "term_id": "GO:0002009",
  "gene_name": "Keratin, type I cuticular Ha8",
  "gene": "UniProtKB:O76015",
  "gene_symbol": "KRT38",
  "term_label": "morphogenesis of an epithelium"
}